regulation of definitive erythrocyte differentiation [GO:0010724] (biological process) Also known as: regulation of definitive RBC differentiation, regulation of definitive erythropoiesis, regulation of definitive red blood cell differentiation Relationships: is a type of regulation of erythrocyte differentiation [GO:0045646]; regulates definitive erythrocyte differentiation [GO:0060318] Sources: GOC:add, GOC:dph, GOC:tb Definition: Any process that modulates the rate, frequency, or extent of definitive erythrocyte differentiation. Definitive erythrocyte differentiation occurs as part of the process of definitive hemopoiesis.